embryonic heart tube formation via epithelial folding [GO:0003145] (biological process) Relationships: is a type of embryonic heart tube formation [GO:0003144] Sources: GOC:mtg_heart Definition: The process that gives rise to the embryonic heart tube by the cells of the heart field along a linear axis.